kinesin binding [GO:0019894] (molecular function) Definition: Interacting selectively and non-covalently and stoichiometrically with kinesin, a member of a superfamily of microtubule-based motor proteins that perform force-generating tasks such as organelle transport and chromosome segregation. References: PMID:8606779 Sources: GOC:curators Relationships: is a type of cytoskeletal protein binding [GO:0008092]